metanephric glomerular mesangial cell differentiation [GO:0072254] (biological process) Sources: GOC:mtg_kidney_jan10 Relationships: is_a glomerular mesangial cell differentiation [GO:0072008]; is a type of metanephric mesangial cell differentiation [GO:0072209]; is part of GO:0072223 Definition: The process in which relatively unspecialized cells acquire specialized structural and/or functional features that characterize the glomerular mesangial cells of the metanephros as it progresses from its formation to the mature state.